{
  "gene_symbol": "TRAF6",
  "term_id": "GO:0043122",
  "gene": "UniProtKB:Q9Y4K3",
  "term_label": "regulation of canonical NF-kappaB signal transduction",
  "gene_name": "TNF receptor-associated factor 6"
}